{
  "gene_name": "SRC kinase signaling inhibitor 1",
  "term_label": "postsynaptic density",
  "gene": "UniProtKB:Q9C0H9",
  "gene_symbol": "SRCIN1",
  "term_id": "GO:0014069"
}